{
  "term_label": "fatty acid elongation, saturated fatty acid",
  "term_id": "GO:0019367",
  "gene": "UniProtKB:A1L3X0",
  "gene_name": "Elongation of very long chain fatty acids protein 7",
  "gene_symbol": "ELOVL7"
}